oxidoreductase activity, acting on CH or CH2 groups, quinone or similar compound as acceptor [GO:0033695] (molecular function) Definition: Catalysis of an oxidation-reduction (redox) reaction in which a CH2 group acts as a hydrogen or electron donor and reduces a quinone or similar acceptor molecule. Sources: EC:1.17.5.-, GOC:mah Subtypes: GO:0033789, GO:0034875, formate dehydrogenase (quinone) activity [GO:0036397] Relationships: is a type of GO:0016725